{
  "term_label": "regulation of immune system process",
  "gene_symbol": "HIC2",
  "term_id": "GO:0002682",
  "gene": "UniProtKB:Q96JB3",
  "gene_name": "Hypermethylated in cancer 2 protein"
}